{
  "term_id": "GO:0019212",
  "term_label": "phosphatase inhibitor activity",
  "gene_name": "Calcineurin B homologous protein 3",
  "gene_symbol": "TESC",
  "gene": "UniProtKB:Q96BS2"
}